{
  "term_label": "Unknown molecular function",
  "gene_symbol": "CCDC32",
  "gene": "UniProtKB:Q9BV29",
  "gene_name": "Coiled-coil domain-containing protein 32",
  "term_id": "UNKNOWN:0001"
}